{
  "term_id": "GO:0004656",
  "term_label": "procollagen-proline 4-dioxygenase activity",
  "gene_name": "Prolyl 4-hydroxylase subunit alpha-1",
  "gene": "UniProtKB:P13674",
  "gene_symbol": "P4HA1"
}